{
  "gene": "UniProtKB:Q9UMR2",
  "gene_name": "ATP-dependent RNA helicase DDX19B",
  "term_label": "mRNA binding",
  "gene_symbol": "DDX19B",
  "term_id": "GO:0003729"
}